{
  "gene_name": "26S proteasome non-ATPase regulatory subunit 10",
  "gene": "UniProtKB:O75832",
  "term_label": "regulation of transcription by RNA polymerase II",
  "term_id": "GO:0006357",
  "gene_symbol": "PSMD10"
}